{
  "gene_name": "Lysozyme-like protein 6",
  "term_label": "lysozyme activity",
  "gene_symbol": "LYZL6",
  "gene": "UniProtKB:O75951",
  "term_id": "GO:0003796"
}